{
  "term_id": "GO:0006955",
  "gene": "UniProtKB:A0A0G2JS06",
  "gene_name": "Immunoglobulin lambda variable 5-39",
  "gene_symbol": "IGLV5-39",
  "term_label": "immune response"
}